{
  "term_label": "glycolytic process",
  "gene": "UniProtKB:P14618",
  "gene_symbol": "PKM",
  "gene_name": "Pyruvate kinase PKM",
  "term_id": "GO:0006096"
}